{
  "term_label": "plasma membrane",
  "term_id": "GO:0005886",
  "gene": "UniProtKB:Q9BX84",
  "gene_name": "Transient receptor potential cation channel subfamily M member 6",
  "gene_symbol": "TRPM6"
}